histone H3R26 methyltransferase activity [GO:0140903] (molecular function) Definition: Catalysis of the reaction: S-adenosyl-L-methionine + (histone H3)-arginine (position 26) = S-adenosyl-L-homocysteine + (histone H3)-N-methyl-arginine (position 26). This reaction is the addition of a methyl group to the arginine residue at position 26 of histone H3. Note: Comment: Note that the residue position corresponds to the canonical human H3 histone (UniProtKB:P84243); this residue is conserved across all eukaryotes. Residue 1 is the first residue following removal of the initiating Methionine (Met). Note that each histone is encoded by multiple genes, and sequences may vary across different genes within an organism. Relationships: is a type of protein-arginine N-methyltransferase activity [GO:0016274]; is a type of histone H3 methyltransferase activity [GO:0140938] Also known as: histone H3R26 arginine methyltransferase activity, histone methylase activity (H3-R26 specific), histone methyltransferase activity (H3-R26 specific), histone-H3R26 methyltransferase activity, histone-arginine N-methyltransferase activity (H3-R26 specific) References: PMID:17882261